{
  "term_label": "regulation of transcription by RNA polymerase II",
  "term_id": "GO:0006357",
  "gene_name": "Ligand-dependent corepressor",
  "gene_symbol": "LCOR",
  "gene": "UniProtKB:Q96JN0"
}